{
  "gene_symbol": "CELF6",
  "gene_name": "CUGBP Elav-like family member 6",
  "term_id": "GO:1990904",
  "gene": "UniProtKB:Q96J87",
  "term_label": "ribonucleoprotein complex"
}